{
  "term_id": "GO:0006357",
  "gene_name": "Zinc finger protein 382",
  "term_label": "regulation of transcription by RNA polymerase II",
  "gene_symbol": "ZNF382",
  "gene": "UniProtKB:Q96SR6"
}